{
  "gene_name": "E3 ubiquitin-protein ligase CBL",
  "gene_symbol": "CBL",
  "gene": "UniProtKB:P22681",
  "term_id": "GO:0007165",
  "term_label": "signal transduction"
}